Golgi reassembly [GO:0090168] (biological process) Relationships: is a type of Golgi organization [GO:0007030]; is a type of cellular component assembly [GO:0022607]; is part of Golgi inheritance [GO:0048313] Definition: The reformation of the Golgi following its breakdown and partitioning contributing to Golgi inheritance. Sources: GOC:ascb_2009, GOC:dph, GOC:tb Also known as: Golgi apparatus reassembly